membrane hyperpolarization [GO:0060081] (biological process) Regulation: regulated by regulation of membrane hyperpolarization [GO:1902630]; negatively regulated by GO:1902631; positively regulated by positive regulation of membrane hyperpolarization [GO:1902632] Sources: GOC:dph Definition: The process in which membrane potential increases with respect to its steady-state potential, usually from negative potential to a more negative potential. For example, during the repolarization phase of an action potential the membrane potential often becomes more negative or hyperpolarized before returning to the steady-state resting potential. Relationships: is_a regulation of membrane potential [GO:0042391]